{
  "gene_name": "Polypeptide N-acetylgalactosaminyltransferase 17",
  "term_label": "Golgi apparatus",
  "gene_symbol": "GALNT17",
  "gene": "UniProtKB:Q6IS24",
  "term_id": "GO:0005794"
}